regulation of cell proliferation involved in mesonephros development [GO:2000606] (biological process) Definition: Any process that modulates the frequency, rate or extent of cell proliferation involved in mesonephros development. Subtypes: regulation of mesonephric glomerular mesangial cell proliferation [GO:2000090], negative regulation of cell proliferation involved in mesonephros development [GO:2000607], positive regulation of cell proliferation involved in mesonephros development [GO:2000608] Relationships: is a type of GO:1901722; regulates cell proliferation involved in mesonephros development [GO:0061209] Sources: GOC:obol